{
  "gene_name": "Fibroblast growth factor 18",
  "term_id": "GO:0005737",
  "term_label": "cytoplasm",
  "gene_symbol": "FGF18",
  "gene": "UniProtKB:O76093"
}